{
  "gene": "UniProtKB:P11831",
  "gene_name": "Serum response factor",
  "term_id": "UNKNOWN:0003",
  "gene_symbol": "SRF",
  "term_label": "Unknown cellular component"
}